{
  "term_id": "UNKNOWN:0002",
  "gene": "UniProtKB:A6NKX1",
  "term_label": "Unknown biological process",
  "gene_symbol": "FAM223B",
  "gene_name": "Protein FAM223B"
}